{
  "term_id": "GO:0005634",
  "gene_symbol": "PITX1",
  "term_label": "nucleus",
  "gene": "UniProtKB:P78337",
  "gene_name": "Pituitary homeobox 1"
}